{
  "gene_symbol": "ZNF702P",
  "term_id": "UNKNOWN:0003",
  "gene": "UniProtKB:Q9H963",
  "gene_name": "Putative zinc finger protein 702",
  "term_label": "Unknown cellular component"
}